{
  "term_id": "UNKNOWN:0001",
  "term_label": "Unknown molecular function",
  "gene_name": "Uncharacterized protein KIAA0087",
  "gene": "UniProtKB:Q14695",
  "gene_symbol": "KIAA0087"
}